folate reductase activity [GO:0033560] (molecular function) Definition: Catalysis of the reaction: 7,8-dihydrofolate + NADP+ = folate + NADPH + H+. Sources: GOC:pde Relationships: is a type of oxidoreductase activity, acting on the CH-NH group of donors, NAD or NADP as acceptor [GO:0016646]